{
  "term_id": "GO:0043529",
  "gene_name": "Guided entry of tail-anchored proteins factor 1",
  "term_label": "GET complex",
  "gene_symbol": "GET1",
  "gene": "UniProtKB:O00258"
}